D-tyrosyl-tRNA(Tyr) deacylase activity [GO:0051500] (molecular function) Relationships: is a type of D-aminoacyl-tRNA deacylase activity [GO:0051499] References: PMID:14527667 Sources: RHEA:25347 Definition: Catalysis of the reaction: D-tyrosyl-tRNATyr + H2O = D-tyrosine + tRNATyr. Removal of a D-tyrosine from a charged tRNA(Tyr).